4-hydroxyphenylacetaldehyde dehydrogenase (NAD+) activity [GO:0047106] (molecular function) Also known as: 4-HPAL dehydrogenase activity, 4-hydroxyphenylacetaldehyde:NAD+ oxidoreductase activity Relationships: is a type of GO:0004029 Sources: RHEA:17273 Definition: Catalysis of the reaction: (4-hydroxyphenyl)acetaldehyde + H2O + NAD+ = 4-hydroxyphenylacetate + 2 H+ + NADH.